{
  "gene": "UniProtKB:Q9UBP8",
  "term_label": "Unknown molecular function",
  "gene_name": "Kidney-associated antigen 1",
  "term_id": "UNKNOWN:0001",
  "gene_symbol": "KAAG1"
}